{
  "gene": "UniProtKB:Q9UDV6",
  "gene_symbol": "ZNF212",
  "gene_name": "Zinc finger protein 212",
  "term_label": "RNA polymerase II cis-regulatory region sequence-specific DNA binding",
  "term_id": "GO:0000978"
}